{
  "gene_symbol": "DAB2",
  "term_id": "GO:0038024",
  "gene": "UniProtKB:P98082",
  "gene_name": "Disabled homolog 2",
  "term_label": "cargo receptor activity"
}